{
  "term_label": "nucleus",
  "gene_symbol": "ADK",
  "gene_name": "Adenosine kinase",
  "term_id": "GO:0005634",
  "gene": "UniProtKB:P55263"
}